{
  "gene_symbol": "TTLL9",
  "term_id": "GO:0000226",
  "gene_name": "Probable tubulin polyglutamylase TTLL9",
  "gene": "UniProtKB:Q3SXZ7",
  "term_label": "microtubule cytoskeleton organization"
}